PCSK9-LDLR complex [GO:1990666] (cellular component) References: PMID:18250299, PMID:24440079 Sources: GOC:BHF, GOC:nc Also known as: PCSK9.LDLR complex, PCSK9/LDL-R complex, PCSK9:low-density lipoprotein receptor complex, PCSK9:EGF-A complex Relationships: is_a protein-containing complex [GO:0032991] Definition: A protein complex consisting of the serine protease PCSK9 (proprotein convertase subtilisin/kexin-9) and a low-density lipoprotein receptor (LDLR). Interaction typically occurs through the epidermal growth factor-like repeat A (EGF-A) domain of the LDLR, and complex formation promotes degradation of the LDLR through the endosome/lysosome pathway.